HRI-mediated signaling [GO:0140468] (biological process) Relationships: is a type of GO:0140467 Also known as: EIF2AK1-mediated signaling References: PMID:27629041 Definition: A series of reactions in which a signal is passed on to downstream proteins within the cell via HRI (also known as EIF2AK1), an intracellular protein kinase that is activated by stress signals, such as heme deficiency, oxidative stress, osmotic shock, mitochondrial dysfunction and heat shock.